{
  "term_id": "GO:0001514",
  "gene_name": "O-phosphoseryl-tRNA(Sec) selenium transferase",
  "term_label": "selenocysteine incorporation",
  "gene_symbol": "SEPSECS",
  "gene": "UniProtKB:Q9HD40"
}